positive regulation of peptidyl-serine phosphorylation [GO:0033138] (biological process) Subtypes: positive regulation of peptidyl-serine phosphorylation of STAT protein [GO:0033141] Definition: Any process that activates or increases the frequency, rate or extent of the phosphorylation of peptidyl-serine. Relationships: is a type of positive regulation of protein phosphorylation [GO:0001934]; is a type of regulation of peptidyl-serine phosphorylation [GO:0033135]; positively regulates GO:0018105 Sources: GOC:mah